dissimilatory sulfate reduction [GO:0019420] (biological process) Relationships: is a type of sulfate assimilation [GO:0000103]; is a type of anaerobic respiration [GO:0009061]; has part GO:0018551 Also known as: dissimilatory sulphate reduction Definition: The reduction of sulfate to hydrogen sulfide, which acts as a terminal electron acceptor. Sulfate is activated to adenosine-phosphosulfate (APS) which is then reduced to sulfite, which is in turn reduced to hydrogen sulfide. References: PMID:25400653, PMID:26680199